{
  "term_id": "GO:0030018",
  "gene": "UniProtKB:Q08043",
  "gene_name": "Alpha-actinin-3",
  "gene_symbol": "ACTN3",
  "term_label": "Z disc"
}